{
  "term_id": "GO:0000978",
  "term_label": "RNA polymerase II cis-regulatory region sequence-specific DNA binding",
  "gene_symbol": "ZNF131",
  "gene": "UniProtKB:P52739",
  "gene_name": "Zinc finger protein 131"
}